peptidyl-glycine modification [GO:0018201] (biological process) Subtypes: N-terminal peptidyl-glycine N-myristoylation [GO:0018008], GO:0018013, peptidyl-1-thioglycine biosynthetic process from peptidyl-glycine [GO:0018173] Relationships: is a type of peptidyl-amino acid modification [GO:0018193] Definition: The modification of peptidyl-glycine. Sources: GOC:go_curators